{
  "term_id": "GO:0043065",
  "gene_symbol": "TRIM35",
  "gene": "UniProtKB:Q9UPQ4",
  "term_label": "positive regulation of apoptotic process",
  "gene_name": "E3 ubiquitin-protein ligase TRIM35"
}